{
  "gene": "UniProtKB:Q9BQB4",
  "gene_name": "Sclerostin",
  "term_id": "GO:0030514",
  "term_label": "negative regulation of BMP signaling pathway",
  "gene_symbol": "SOST"
}